{
  "term_label": "negative regulation of synaptic transmission, dopaminergic",
  "gene": "UniProtKB:P20382",
  "term_id": "GO:0032227",
  "gene_symbol": "PMCH",
  "gene_name": "Pro-MCH"
}